endodeoxyribonuclease activator activity [GO:0140656] (molecular function) Definition: Binds to and increases the activity of an endodeoxyribonuclease. Subtypes: single-stranded DNA endodeoxyribonuclease activator activity [GO:1990600] References: PMID:33836577 Relationships: is a type of nuclease activator activity [GO:0170053]; positively regulates DNA endonuclease activity [GO:0004520]